positive regulation of mitochondrial calcium ion concentration [GO:0051561] (biological process) Also known as: elevation of calcium ion concentration in mitochondria, elevation of calcium ion concentration in mitochondrion, elevation of mitochondrial calcium ion concentration, mitochondrial calcium ion concentration elevation Relationships: is_a mitochondrial calcium ion homeostasis [GO:0051560] Sources: GOC:ai Definition: Any process that increases the concentration of calcium ions in mitochondria.